{
  "gene_name": "G1_S-specific cyclin-D3",
  "term_label": "cyclin-dependent protein serine/threonine kinase regulator activity",
  "term_id": "GO:0016538",
  "gene_symbol": "CCND3",
  "gene": "UniProtKB:P30281"
}